{
  "gene_name": "Kelch-like protein 31",
  "term_id": "UNKNOWN:0001",
  "gene": "UniProtKB:Q9H511",
  "gene_symbol": "KLHL31",
  "term_label": "Unknown molecular function"
}